{
  "gene_symbol": "TNFRSF1B",
  "gene": "UniProtKB:P20333",
  "term_id": "GO:0008630",
  "term_label": "intrinsic apoptotic signaling pathway in response to DNA damage",
  "gene_name": "Tumor necrosis factor receptor superfamily member 1B"
}